{
  "gene_symbol": "HTR1F",
  "gene": "UniProtKB:P30939",
  "gene_name": "5-hydroxytryptamine receptor 1F",
  "term_label": "neurotransmitter receptor activity",
  "term_id": "GO:0030594"
}